positive regulation of cellulosome assembly [GO:1900505] (biological process) Also known as: up regulation of cellulosome assembly, up-regulation of cellulosome assembly, upregulation of cellulosome assembly, activation of cellulosome assembly Sources: GOC:TermGenie, GOC:mengo_curators Relationships: is a type of regulation of cellulosome assembly [GO:1900503]; is a type of positive regulation of organelle assembly [GO:1902117]; positively regulates cellulosome assembly [GO:0044575] Definition: Any process that activates or increases the frequency, rate or extent of cellulosome assembly.